{
  "gene_name": "Short transient receptor potential channel 5",
  "gene_symbol": "TRPC5",
  "gene": "UniProtKB:Q9UL62",
  "term_label": "store-operated calcium channel activity",
  "term_id": "GO:0015279"
}